single-stranded DNA 3'-5' DNA exonuclease activity [GO:0008310] (molecular function) Also known as: single-stranded DNA 3'-5' exodeoxyribonuclease activity, exonuclease I activity, single-stranded DNA specific 3'-5' exodeoxyribonuclease activity, ssDNA-specific 3'-5' exodeoxyribonuclease activity Definition: Catalysis of the sequential cleavage of mononucleotides from a free 3' terminus of a single-stranded DNA molecule. Relationships: is a type of 3'-5'-DNA exonuclease activity [GO:0008296]; is a type of single-stranded DNA exodeoxyribonuclease activity [GO:0008297] References: PMID:22562358 Sources: GOC:mah